{
  "gene_name": "DNA polymerase zeta catalytic subunit",
  "term_id": "GO:0042276",
  "gene_symbol": "REV3L",
  "term_label": "error-prone translesion synthesis",
  "gene": "UniProtKB:O60673"
}